{
  "gene": "UniProtKB:P10276",
  "term_id": "GO:0004879",
  "gene_symbol": "RARA",
  "term_label": "nuclear receptor activity",
  "gene_name": "Retinoic acid receptor alpha"
}